{
  "gene_name": "Prostaglandin E2 receptor EP2 subtype",
  "term_id": "GO:0004957",
  "gene": "UniProtKB:P43116",
  "gene_symbol": "PTGER2",
  "term_label": "prostaglandin E receptor activity"
}